{
  "term_id": "GO:0044325",
  "gene_symbol": "LRRC38",
  "gene_name": "Leucine-rich repeat-containing protein 38",
  "gene": "UniProtKB:Q5VT99",
  "term_label": "transmembrane transporter binding"
}